{
  "gene_symbol": "ASF1B",
  "term_id": "GO:0005634",
  "term_label": "nucleus",
  "gene_name": "Histone chaperone ASF1B",
  "gene": "UniProtKB:Q9NVP2"
}